pigment biosynthetic process involved in pigment granule maturation [GO:0048784] (biological process) Relationships: is a type of pigment metabolic process involved in developmental pigmentation [GO:0043324]; is a type of pigment biosynthetic process involved in pigment accumulation [GO:0043477]; is part of GO:0048757 Sources: GOC:jid Definition: The chemical reactions and pathways resulting in the formation of a pigment, contributing to the process in which a membrane-bounded organelle develops into a pigment granule. Maturation is a developmental process, independent of morphogenetic (shape) change, that is required for a cell or structure to attain its fully functional state. Also known as: pigment biosynthetic process during pigment granule maturation